{
  "gene_symbol": "CADPS",
  "term_id": "GO:0045921",
  "gene": "UniProtKB:Q9ULU8",
  "term_label": "positive regulation of exocytosis",
  "gene_name": "Calcium-dependent secretion activator 1"
}